{
  "term_id": "UNKNOWN:0003",
  "gene_symbol": "C10orf53",
  "term_label": "Unknown cellular component",
  "gene": "UniProtKB:Q8N6V4",
  "gene_name": "UPF0728 protein C10orf53"
}